{
  "term_label": "CHRAC",
  "gene_symbol": "CHRAC1",
  "gene": "UniProtKB:Q9NRG0",
  "gene_name": "Chromatin accessibility complex protein 1",
  "term_id": "GO:0008623"
}